{
  "gene_name": "Sodium- and chloride-dependent GABA transporter 2",
  "gene": "UniProtKB:Q9NSD5",
  "term_id": "GO:0005886",
  "gene_symbol": "SLC6A13",
  "term_label": "plasma membrane"
}